{
  "gene_symbol": "ADAMTS10",
  "gene": "UniProtKB:Q9H324",
  "term_label": "extracellular matrix",
  "term_id": "GO:0031012",
  "gene_name": "A disintegrin and metalloproteinase with thrombospondin motifs 10"
}